{
  "gene_name": "Guanine nucleotide-binding protein G(T) subunit gamma-T1",
  "gene_symbol": "GNGT1",
  "term_id": "GO:0007186",
  "term_label": "G protein-coupled receptor signaling pathway",
  "gene": "UniProtKB:P63211"
}